{
  "gene_symbol": "TRIM21",
  "term_id": "GO:0010508",
  "term_label": "positive regulation of autophagy",
  "gene": "UniProtKB:P19474",
  "gene_name": "E3 ubiquitin-protein ligase TRIM21"
}